{
  "term_label": "olfactory receptor activity",
  "gene_name": "Olfactory receptor 4C3",
  "gene": "UniProtKB:Q8NH37",
  "gene_symbol": "OR4C3",
  "term_id": "GO:0004984"
}